{
  "term_label": "microtubule cytoskeleton organization",
  "gene_name": "Partitioning defective 3 homolog B",
  "term_id": "GO:0000226",
  "gene_symbol": "PARD3B",
  "gene": "UniProtKB:Q8TEW8"
}